{
  "gene_symbol": "VWA2",
  "term_id": "UNKNOWN:0001",
  "term_label": "Unknown molecular function",
  "gene": "UniProtKB:Q5GFL6",
  "gene_name": "von Willebrand factor A domain-containing protein 2"
}